negative regulation of response to external stimulus [GO:0032102] (biological process) Definition: Any process that stops, prevents, or reduces the frequency, rate or extent of a response to an external stimulus. Sources: GOC:mah Also known as: down regulation of response to external stimulus, down-regulation of response to external stimulus, downregulation of response to external stimulus, inhibition of response to external stimulus Note: Note that this term is in the subset of terms that should not be used for direct gene product annotation. Instead, select a child term or, if no appropriate child term exists, please request a new term. Direct annotations to this term may be amended during annotation QC. Relationships: is a type of GO:0032101; is a type of negative regulation of response to stimulus [GO:0048585]; negatively regulates response to external stimulus [GO:0009605] Subtypes: negative regulation of antimicrobial humoral response [GO:0008348], negative regulation of systemic acquired resistance [GO:0010113], negative regulation of opsin-mediated signaling pathway [GO:0016059], negative regulation of lipopolysaccharide-mediated signaling pathway [GO:0031665], negative regulation of innate immune response [GO:0045824], GO:0048681, negative regulation of defense response to virus [GO:0050687], negative regulation of inflammatory response [GO:0050728], negative regulation of chemotaxis [GO:0050922], prepulse inhibition [GO:0060134], negative regulation of wound healing [GO:0061045], GO:0070955, negative regulation of defense response to insect [GO:1900366], negative regulation of defense response to bacterium [GO:1900425], negative regulation of defense response to oomycetes [GO:1902289], negative regulation of chemokinesis [GO:1904366], negative regulation of xenophagy [GO:1904416], negative regulation of detection of mechanical stimulus involved in sensory perception of touch [GO:1905788], negative regulation of mechanosensory behavior [GO:1905791]